laminin-522 complex [GO:1990339] (CC) Relationships: is a type of laminin complex [GO:0043256] Definition: A laminin complex composed of alpha5, beta2 and gamma2 polypeptide chains. Also known as: laminin-522 References: PMID:15979864, PMID:17453709 Sources: GOC:bhm, GOC:dph